{
  "gene_name": "SWI_SNF-related matrix-associated actin-dependent regulator of chromatin subfamily A containing DEAD_H box 1",
  "gene": "UniProtKB:Q9H4L7",
  "term_label": "positive regulation of transcription by RNA polymerase II",
  "gene_symbol": "SMARCAD1",
  "term_id": "GO:0045944"
}